{
  "gene": "UniProtKB:Q9H0U6",
  "term_id": "GO:0005739",
  "gene_symbol": "MRPL18",
  "term_label": "mitochondrion",
  "gene_name": "Large ribosomal subunit protein uL18m"
}